{
  "gene_name": "Leucine-rich repeat and calponin homology domain-containing protein 1",
  "gene_symbol": "LRCH1",
  "term_label": "cellular response to chemokine",
  "term_id": "GO:1990869",
  "gene": "UniProtKB:Q9Y2L9"
}